{
  "gene_symbol": "NOXO1",
  "gene": "UniProtKB:Q8NFA2",
  "gene_name": "NADPH oxidase organizer 1",
  "term_id": "GO:0005737",
  "term_label": "cytoplasm"
}